{
  "term_label": "nucleoside diphosphate kinase activity",
  "term_id": "GO:0004550",
  "gene": "UniProtKB:Q5TCS8",
  "gene_name": "Adenylate kinase 9",
  "gene_symbol": "AK9"
}